{
  "term_label": "positive regulation of neuron projection development",
  "gene_symbol": "DDR2",
  "gene": "UniProtKB:Q16832",
  "gene_name": "Discoidin domain-containing receptor 2",
  "term_id": "GO:0010976"
}